{
  "term_id": "GO:0005886",
  "gene": "UniProtKB:Q8N0Z9",
  "term_label": "plasma membrane",
  "gene_name": "V-set and immunoglobulin domain-containing protein 10",
  "gene_symbol": "VSIG10"
}